{
  "term_id": "UNKNOWN:0002",
  "term_label": "Unknown biological process",
  "gene_symbol": "MATK",
  "gene_name": "Megakaryocyte-associated tyrosine-protein kinase",
  "gene": "UniProtKB:P42679"
}